L-phenylalanine N-acetyltransferase activity [GO:0050176] (molecular function) Also known as: phenylalanine N-acetyltransferase activity, acetyl-CoA-L-phenylalanine alpha-N-acetyltransferase activity, acetyl-CoA:L-phenylalanine N-acetyltransferase activity Relationships: is a type of L-amino-acid N-acetyltransferase activity [GO:0140085] Sources: EC:2.3.1.53, RHEA:17801 Definition: Catalysis of the reaction: L-phenylalanine + acetyl-CoA = N-acetyl-L-phenylalanine + CoA + H+.